mannose:proton symporter activity [GO:0055053] (molecular function) Definition: Enables the transfer of a solute or solutes from one side of a membrane to the other according to the reaction: mannose + H+ = mannose + H+. Sources: GOC:ct Also known as: mannose:hydrogen symporter activity Relationships: is a type of hexose:proton symporter activity [GO:0009679]; is a type of mannose transmembrane transporter activity [GO:0015578]